ruffle [GO:0001726] (cellular component) Relationships: is a type of plasma membrane bounded cell projection [GO:0120025]; is part of cell leading edge [GO:0031252] Definition: Projection at the leading edge of a crawling cell; the protrusions are supported by a microfilament meshwork. Also known as: membrane ruffle Sources: ISBN:0124325653